{
  "term_label": "negative regulation of T cell mediated cytotoxicity",
  "term_id": "GO:0001915",
  "gene_symbol": "KLRC1",
  "gene": "UniProtKB:P26715",
  "gene_name": "NKG2-A_NKG2-B type II integral membrane protein"
}